alpha-methylacyl-CoA racemase activity [GO:0008111] (molecular function) Definition: Catalysis of the reaction: (2S)-2-methylacyl-CoA = (2R)-2-methylacyl-CoA. Sources: EC:5.1.99.4 Also known as: 2-methylacyl-CoA 2-epimerase activity Relationships: is a type of racemase and epimerase activity [GO:0016854]